gonadotropin hormone-releasing hormone activity [GO:0005183] (molecular function) Definition: The action characteristic of gonadotropin hormone-releasing hormone (GnRH), any of a family of decapeptide amide hormones that are released by the hypothalamus in response to neural and/or chemical stimuli. In at least mammals, upon receptor binding, GnRH causes the release of follicle-stimulating hormone (FSH) and luteinizing hormone (LH) by the anterior pituitary. References: PMID:11026571 Sources: ISBN:0198506732, Wikipedia:Gonadotropin-releasing_hormone Also known as: GnRH activity, LH/FSH-RF, LHRH activity, gonadotrophin hormone-releasing hormone activity, luteinizing hormone-releasing factor activity, luteinizing hormone-releasing hormone activity, luteinizing hormone/follicle-stimulating hormone releasing factor activity Relationships: is_a GO:0005179